{
  "gene_symbol": "KIFC2",
  "term_label": "axon guidance",
  "term_id": "GO:0007411",
  "gene_name": "Kinesin-like protein KIFC2",
  "gene": "UniProtKB:Q96AC6"
}